fatty acid elongation, polyunsaturated fatty acid [GO:0034626] (biological process) Sources: GOC:mah Relationships: is a type of fatty acid elongation, unsaturated fatty acid [GO:0019368] Definition: Elongation of a fatty acid chain into which two or more C-C double bonds have been introduced.